regulation of retrograde vesicle-mediated transport, Golgi to ER [GO:2000156] (biological process) Relationships: is a type of regulation of vesicle-mediated transport [GO:0060627]; regulates retrograde vesicle-mediated transport, Golgi to endoplasmic reticulum [GO:0006890] Definition: Any process that modulates the frequency, rate or extent of retrograde vesicle-mediated transport, Golgi to ER. Sources: GOC:mah Also known as: regulation of cis-Golgi to rough ER transport, regulation of cis-Golgi to rough ER vesicle-mediated transport, regulation of cis-Golgi to rough endoplasmic reticulum transport, regulation of cis-Golgi to rough endoplasmic reticulum vesicle-mediated transport, regulation of retrograde (Golgi to ER) transport, regulation of retrograde transport, Golgi to ER, regulation of retrograde transport, Golgi to endoplasmic reticulum, regulation of retrograde vesicle-mediated transport, Golgi to endoplasmic reticulum